{
  "gene": "UniProtKB:Q16518",
  "term_id": "GO:0052885",
  "gene_symbol": "RPE65",
  "gene_name": "Retinoid isomerohydrolase",
  "term_label": "all-trans-retinyl-ester hydrolase, 11-cis retinol forming activity"
}